{
  "gene_name": "Arachidonate 12-lipoxygenase, 12R-type",
  "term_label": "arachidonate metabolic process",
  "gene_symbol": "ALOX12B",
  "gene": "UniProtKB:O75342",
  "term_id": "GO:0019369"
}